{
  "gene_symbol": "PDLIM1",
  "gene": "UniProtKB:O00151",
  "term_label": "Z disc",
  "term_id": "GO:0030018",
  "gene_name": "PDZ and LIM domain protein 1"
}